{
  "term_id": "UNKNOWN:0001",
  "gene": "UniProtKB:Q07654",
  "gene_symbol": "TFF3",
  "gene_name": "Trefoil factor 3",
  "term_label": "Unknown molecular function"
}